natural killer cell mediated immunity [GO:0002228] (biological process) Definition: The promotion of an immune response by natural killer cells through direct recognition of target cells or through the release of cytokines. Subtypes: natural killer cell cytokine production [GO:0002370], natural killer cell mediated immune response to tumor cell [GO:0002423], natural killer cell mediated cytotoxicity [GO:0042267] Also known as: NK cell mediated immunity Sources: GOC:add, GO_REF:0000022, ISBN:0781735149 Regulation: RO_0002211 by regulation of natural killer cell mediated immunity [GO:0002715]; negatively regulated by negative regulation of natural killer cell mediated immunity [GO:0002716]; positively regulated by positive regulation of natural killer cell mediated immunity [GO:0002717] Relationships: is a type of GO:0002449; is a type of GO:0045087